{
  "gene_name": "Potassium voltage-gated channel subfamily A member 4",
  "term_id": "GO:0008076",
  "gene_symbol": "KCNA4",
  "term_label": "voltage-gated potassium channel complex",
  "gene": "UniProtKB:P22459"
}